{
  "gene_name": "Uncharacterized protein",
  "gene": "UniProtKB:A0A1B0GTQ1",
  "gene_symbol": "A0A1B0GTQ1",
  "term_id": "UNKNOWN:0001",
  "term_label": "Unknown molecular function"
}